glycolate transmembrane transport [GO:0097339] (biological process) Relationships: is_a glycolate transport [GO:1900866]; is a type of GO:1905039 Note: Note that this term is not intended for use in annotating lateral movement within membranes. Also known as: glycolate membrane transport Definition: The process in which glycolate is transported across a membrane. Glycolate is the anion of hydroxyethanoic acid (glycolic acid). References: PMID:11283302, PMID:11785976 Sources: GOC:am